positive regulation of extracellular exosome assembly [GO:1903553] (biological process) Definition: Any process that activates or increases the frequency, rate or extent of extracellular vesicular exosome assembly. References: PMID:24105262 Sources: GOC:TermGenie, GO_REF:0000058 Also known as: up regulation of extracellular vesicular exosome assembly, up-regulation of extracellular vesicular exosome assembly, upregulation of extracellular vesicular exosome assembly, activation of extracellular vesicular exosome assembly, positive regulation of extracellular vesicular exosome assembly Relationships: is a type of positive regulation of organelle assembly [GO:1902117]; is a type of GO:1903551; positively regulates extracellular exosome assembly [GO:0071971]